{
  "gene": "UniProtKB:O95995",
  "term_label": "axoneme assembly",
  "term_id": "GO:0035082",
  "gene_symbol": "GAS8",
  "gene_name": "Dynein regulatory complex subunit 4"
}